ceramide 1-phosphate binding [GO:1902387] (molecular function) Relationships: is_a phospholipid binding [GO:0005543]; is_a anion binding [GO:0043168]; is a type of ceramide binding [GO:0097001] References: PMID:23863933 Sources: GOC:TermGenie Definition: Binding to ceramide 1-phosphate.